{
  "gene_symbol": "HAP1",
  "gene_name": "Huntingtin-associated protein 1",
  "term_label": "dendrite",
  "gene": "UniProtKB:P54257",
  "term_id": "GO:0030425"
}